{
  "term_label": "protein serine/threonine phosphatase activity",
  "gene": "UniProtKB:P60510",
  "term_id": "GO:0004722",
  "gene_symbol": "PPP4C",
  "gene_name": "Serine_threonine-protein phosphatase 4 catalytic subunit"
}